{
  "gene": "UniProtKB:Q8NDB6",
  "term_id": "UNKNOWN:0001",
  "term_label": "Unknown molecular function",
  "gene_name": "Protein FAM156A_FAM156B",
  "gene_symbol": "FAM156B"
}